2-keto-3-deoxygalactonate aldolase activity [GO:0043724] (molecular function) Relationships: is a type of GO:0016836 Also known as: KDGal aldolase activity Definition: Catalysis of the reaction: 2-keto-3-deoxygalactonate = D-glyceraldehyde + pyruvate. References: PMID:12824170